{
  "gene_symbol": "STK17A",
  "term_label": "protein serine/threonine kinase activity",
  "gene_name": "Serine_threonine-protein kinase 17A",
  "term_id": "GO:0004674",
  "gene": "UniProtKB:Q9UEE5"
}